positive regulation of basidiospore formation [GO:0075303] (BP) Relationships: is a type of GO:0043941; is a type of GO:0075302; positively regulates basidiospore formation [GO:0034295] Sources: GOC:pamgo_curators Definition: Any process that activates, maintains or increases the frequency, rate or extent of frequency, rate or extent of basidiospore formation, a process in which a sexually produced fungal spore is formed on a basidium in the fungi basidiomycetes.